{
  "gene_name": "Phospholipid-transporting ATPase VA",
  "term_id": "GO:0005886",
  "gene_symbol": "ATP10A",
  "term_label": "plasma membrane",
  "gene": "UniProtKB:O60312"
}